{
  "term_id": "GO:0030855",
  "gene_name": "Uroplakin-2",
  "term_label": "epithelial cell differentiation",
  "gene": "UniProtKB:O00526",
  "gene_symbol": "UPK2"
}